{
  "gene_symbol": "TM2D1",
  "term_label": "apoptotic signaling pathway",
  "gene": "UniProtKB:Q9BX74",
  "term_id": "GO:0097190",
  "gene_name": "TM2 domain-containing protein 1"
}